{
  "gene": "UniProtKB:P01601",
  "term_label": "Unknown molecular function",
  "gene_name": "Immunoglobulin kappa variable 1D-16",
  "gene_symbol": "IGKV1D-16",
  "term_id": "UNKNOWN:0001"
}